{
  "term_id": "GO:0048306",
  "gene": "UniProtKB:P31949",
  "gene_symbol": "S100A11",
  "term_label": "calcium-dependent protein binding",
  "gene_name": "Protein S100-A11"
}